{
  "gene_symbol": "ASL",
  "gene_name": "Argininosuccinate lyase",
  "term_label": "L-arginine biosynthetic process via ornithine",
  "term_id": "GO:0042450",
  "gene": "UniProtKB:P04424"
}